nitrogen catabolite activation of transcription [GO:0090294] (biological process) References: PMID:19104072 Sources: GOC:mah, GOC:rb Relationships: is_a positive regulation of DNA-templated transcription [GO:0045893]; is a type of GO:0090293 Subtypes: GO:0001080 Also known as: positive regulation of transcription by nitrogen catabolites Definition: A transcription regulation process in which the presence of one nitrogen source leads to an increase in the frequency, rate, or extent of transcription of specific genes involved in the metabolism of other nitrogen sources.